{
  "gene_symbol": "SFXN5",
  "term_id": "GO:1990542",
  "gene_name": "Sideroflexin-5",
  "gene": "UniProtKB:Q8TD22",
  "term_label": "mitochondrial transmembrane transport"
}